GCU codon-amino acid adaptor activity [GO:0033453] (molecular function) Note: Note that in the standard genetic code, GCT codes for alanine. Sources: GOC:mah Relationships: is a type of triplet codon-amino acid adaptor activity [GO:0030533] Definition: A triplet codon-amino acid adaptor activity that recognizes a GCU codon. Also known as: GCT codon-amino acid adaptor activity, alanine tRNA